{
  "term_id": "GO:0005886",
  "gene_symbol": "PMP22",
  "gene": "UniProtKB:Q01453",
  "term_label": "plasma membrane",
  "gene_name": "Peripheral myelin protein 22"
}